guanosine salvage [GO:0006179] (biological process) Sources: GOC:jl Relationships: is a type of purine ribonucleoside salvage [GO:0006166]; is a type of guanosine biosynthetic process [GO:0046114] Also known as: guanine, xanthine and their nucleoside salvage Definition: Any process that generates guanosine, guanine riboside, from derivatives of it without de novo synthesis.